{
  "gene": "UniProtKB:Q96NL8",
  "gene_symbol": "CFAP418",
  "term_label": "Unknown molecular function",
  "gene_name": "Cilia- and flagella-associated protein 418",
  "term_id": "UNKNOWN:0001"
}